caste determination, influence by environmental factors [GO:0048650] (biological process) Relationships: is a type of caste determination [GO:0048648]; is a type of polyphenic determination, influence by environmental factors [GO:0048651] Sources: GOC:jid Definition: The process in which individuals, having the potential to develop any of several distinct developmental paths, have their individual developmental fate determined in response to environmental cues. Individuals with distinct developmental fates perform different functions in a colony of social insects.